{
  "gene_symbol": "RPS16",
  "term_label": "RNA binding",
  "gene": "UniProtKB:P62249",
  "gene_name": "Small ribosomal subunit protein uS9",
  "term_id": "GO:0003723"
}